{
  "gene_name": "Low-density lipoprotein receptor class A domain-containing protein 1",
  "gene": "UniProtKB:Q5T700",
  "term_id": "UNKNOWN:0002",
  "term_label": "Unknown biological process",
  "gene_symbol": "LDLRAD1"
}